{
  "term_label": "plasma membrane",
  "gene": "UniProtKB:Q15825",
  "term_id": "GO:0005886",
  "gene_symbol": "CHRNA6",
  "gene_name": "Neuronal acetylcholine receptor subunit alpha-6"
}